{
  "gene": "UniProtKB:Q9UL49",
  "term_label": "regulation of DNA-templated transcription",
  "gene_symbol": "TCFL5",
  "term_id": "GO:0006355",
  "gene_name": "Transcription factor-like 5 protein"
}